{
  "gene_symbol": "THOC6",
  "term_label": "mRNA export from nucleus",
  "term_id": "GO:0006406",
  "gene": "UniProtKB:Q86W42",
  "gene_name": "THO complex subunit 6 homolog"
}